intranuclear rod assembly [GO:1905861] (biological process) Definition: The aggregation, arrangement and bonding together of a set of components to form an intranuclear rod. References: PMID:28074884 Sources: GOC:TermGenie, GO_REF:0000079 Also known as: intranuclear actin rod assembly, intranuclear actin rod formation, intranuclear rod formation Relationships: is a type of cellular component assembly [GO:0022607]; is a type of supramolecular fiber organization [GO:0097435]